{
  "gene_name": "LEM domain-containing protein 1",
  "gene_symbol": "LEMD1",
  "gene": "UniProtKB:Q68G75",
  "term_id": "UNKNOWN:0001",
  "term_label": "Unknown molecular function"
}